{
  "gene_symbol": "VCX3A",
  "gene_name": "Variable charge X-linked protein 3",
  "gene": "UniProtKB:Q9NNX9",
  "term_label": "brain development",
  "term_id": "GO:0007420"
}